ESCRT III complex [GO:0000815] (cellular component) Definition: A complex with membrane scission activity that plays a major role in many processes where membranes are remodelled - including endosomal transport (vesicle budding), nuclear envelope organisation (membrane closure, mitotic bridge cleavage), and cytokinesis (abscission). Also known as: endosomal sorting complex required for transport References: PMID:17556548, PMID:22361144, PMID:28242692, PMID:31132588, PMID:32243490, PMID:34449766 Relationships: is a type of GO:0036452; is a type of membrane protein complex [GO:0098796]; is part of endosome membrane [GO:0010008]